{
  "gene": "UniProtKB:Q9UJ99",
  "gene_symbol": "CDH22",
  "term_label": "cadherin binding",
  "gene_name": "Cadherin-22",
  "term_id": "GO:0045296"
}